{
  "gene_name": "Protein FAM229B",
  "gene_symbol": "FAM229B",
  "term_label": "Unknown biological process",
  "gene": "UniProtKB:Q4G0N7",
  "term_id": "UNKNOWN:0002"
}